{
  "gene_symbol": "BOK",
  "gene_name": "Bcl-2-related ovarian killer protein",
  "term_id": "GO:0005741",
  "term_label": "mitochondrial outer membrane",
  "gene": "UniProtKB:Q9UMX3"
}